{
  "term_label": "plasma membrane",
  "term_id": "GO:0005886",
  "gene_symbol": "CSNK1G1",
  "gene": "UniProtKB:Q9HCP0",
  "gene_name": "Casein kinase I isoform gamma-1"
}